{
  "term_label": "valine-tRNA ligase activity",
  "gene_symbol": "VARS2",
  "term_id": "GO:0004832",
  "gene": "UniProtKB:Q5ST30",
  "gene_name": "Valine--tRNA ligase, mitochondrial"
}